{
  "term_id": "GO:0003677",
  "gene_symbol": "YAF2",
  "term_label": "DNA binding",
  "gene_name": "YY1-associated factor 2",
  "gene": "UniProtKB:Q8IY57"
}